{
  "gene_name": "NUT family member 1",
  "term_id": "UNKNOWN:0001",
  "gene": "UniProtKB:Q86Y26",
  "term_label": "Unknown molecular function",
  "gene_symbol": "NUTM1"
}